polyribonucleotide nucleotidyltransferase activity [GO:0004654] (molecular function) Sources: EC:2.7.7.8 Also known as: nucleoside diphosphate:polynucleotidyl transferase activity, polynucleotide phosphorylase activity, polyribonucleotide phosphorylase activity, polyribonucleotide:phosphate nucleotidyltransferase activity Definition: Catalysis of the reaction: RNA(n+1) + phosphate = RNA(n) + a nucleoside diphosphate. Relationships: is a type of nucleotidyltransferase activity [GO:0016779]